{
  "term_id": "GO:0005886",
  "gene_symbol": "TRBV30",
  "term_label": "plasma membrane",
  "gene": "UniProtKB:A0A0K0K1B3",
  "gene_name": "T cell receptor beta variable 30"
}